{
  "term_id": "GO:0010833",
  "gene_name": "CST complex subunit STN1",
  "gene_symbol": "STN1",
  "gene": "UniProtKB:Q9H668",
  "term_label": "telomere maintenance via telomere lengthening"
}